{
  "gene_symbol": "LST1",
  "term_label": "membrane",
  "gene": "UniProtKB:O00453",
  "term_id": "GO:0016020",
  "gene_name": "Leukocyte-specific transcript 1 protein"
}